negative regulation of oomycete sporangium development [GO:0075324] (biological process) Definition: Any process that stops, prevents, or reduces the frequency, rate or extent of oomycete sporangium development, a process that leads to the formation of oomycete sporangium, a single-celled or many-celled structure that germinates directly to form an infection hypha or differentiate, through specialized cleavage vesicles, into between 10 and 30 zoospores, which is laterally flagellated. Relationships: is a type of negative regulation of sporulation [GO:0043939]; is a type of negative regulation of sporangium development [GO:0075312]; is a type of regulation of oomycete sporangium development [GO:0075322]; is a type of negative regulation of asexual reproduction [GO:1903665]; negatively regulates oomycete sporangium development [GO:0075321] Sources: GOC:pamgo_curators